{
  "gene": "UniProtKB:Q86YD1",
  "term_id": "GO:0005667",
  "term_label": "transcription regulator complex",
  "gene_name": "Prostate tumor-overexpressed gene 1 protein",
  "gene_symbol": "PTOV1"
}